{
  "gene_symbol": "WNT5B",
  "gene_name": "Protein Wnt-5b",
  "term_label": "cytokine activity",
  "term_id": "GO:0005125",
  "gene": "UniProtKB:Q9H1J7"
}